spermidine hydroxycinnamate conjugate biosynthetic process [GO:0080088] (biological process) Definition: The chemical reactions and pathways resulting in the formation of spermidine hydroxycinnamate conjugates. Relationships: is a type of amide biosynthetic process [GO:0043604] References: PMID:19077165